mitochondrial depolarization [GO:0051882] (biological process) Relationships: is a type of GO:0051881; is a type of membrane depolarization [GO:0051899]; occurs in GO:0005739 Sources: Wikipedia:Depolarization, Wikipedia:Mitochondrion Also known as: mitochondria depolarization, mitochondrial depolarisation, mitochondrial membrane depolarization, mitochondrion depolarization Definition: The process in which the potential difference across the mitochondrial membrane is reduced from its steady state level. Regulation: regulated by GO:0051900; positively regulated by positive regulation of mitochondrial depolarization [GO:0051901]; negatively regulated by negative regulation of mitochondrial depolarization [GO:0051902]